{
  "gene": "UniProtKB:Q00532",
  "gene_symbol": "CDKL1",
  "gene_name": "Cyclin-dependent kinase-like 1",
  "term_id": "UNKNOWN:0002",
  "term_label": "Unknown biological process"
}